{
  "gene_name": "Guanine nucleotide-binding protein G(s) subunit alpha isoforms XLas",
  "term_label": "GTPase activity",
  "gene": "UniProtKB:Q5JWF2",
  "term_id": "GO:0003924",
  "gene_symbol": "GNAS"
}